{
  "gene_symbol": "SLC9B1P1",
  "term_id": "UNKNOWN:0003",
  "gene": "UniProtKB:A6NJY1",
  "term_label": "Unknown cellular component",
  "gene_name": "Putative SLC9B1-like protein SLC9B1P1"
}